nuclear localization sequence binding [GO:0008139] (molecular function) Also known as: NLS binding, nuclear localisation sequence binding, nuclear localization signal binding Sources: GOC:ai Definition: Binding to a nuclear localization sequence, a specific peptide sequence that acts as a signal to localize the protein within the nucleus. Relationships: is a type of signal sequence binding [GO:0005048]